RNA lariat debranching enzyme activator activity [GO:0061632] (molecular function) References: PMID:24919400 Sources: GOC:dph Definition: Binds to and increases the activity of an RNA lariat debranching enzyme. Relationships: is a type of ribonuclease activator activity [GO:0170054]; positively regulates GO:0008419